{
  "gene_symbol": "ARHGEF25",
  "term_label": "cytoplasm",
  "gene_name": "Rho guanine nucleotide exchange factor 25",
  "term_id": "GO:0005737",
  "gene": "UniProtKB:Q86VW2"
}